{
  "gene_symbol": "PRPS1L1",
  "term_id": "GO:0004749",
  "gene_name": "Ribose-phosphate pyrophosphokinase 3",
  "gene": "UniProtKB:P21108",
  "term_label": "ribose phosphate diphosphokinase activity"
}